{
  "term_id": "GO:0006027",
  "gene_name": "N-sulphoglucosamine sulphohydrolase",
  "term_label": "glycosaminoglycan catabolic process",
  "gene_symbol": "SGSH",
  "gene": "UniProtKB:P51688"
}